leading edge cell fate commitment [GO:0035027] (biological process) Definition: The commitment of cells to leading edge cell fate and their capacity to differentiate into leading edge cells. Leading edge cells are found at the front of a migrating epithelial sheet. Sources: GOC:bf Relationships: is a type of epithelial cell fate commitment [GO:0072148]; is part of GO:0035026 Subtypes: dorsal closure, leading edge cell fate commitment [GO:0035029]